{
  "term_id": "GO:0001772",
  "term_label": "immunological synapse",
  "gene": "UniProtKB:O43561",
  "gene_name": "Linker for activation of T-cells family member 1",
  "gene_symbol": "LAT"
}